detection of gravity [GO:0009590] (biological process) Relationships: is a type of detection of external stimulus [GO:0009581]; is a type of detection of abiotic stimulus [GO:0009582]; is_a response to gravity [GO:0009629] Subtypes: GO:0070999 Also known as: perception of gravity Definition: The series of events in which a gravitational stimulus is received and converted into a molecular signal. Sources: GOC:dos, GOC:hb